{
  "gene": "UniProtKB:O60488",
  "term_id": "GO:0005811",
  "term_label": "lipid droplet",
  "gene_name": "Long-chain-fatty-acid--CoA ligase 4",
  "gene_symbol": "ACSL4"
}